2-methylbutanoyl-CoA(4-) catabolic process [GO:1902190] (biological process) References: PMID:15574432 Sources: GOC:TermGenie Also known as: 2-methylbutanoyl-CoA(4-) breakdown, 2-methylbutanoyl-CoA(4-) catabolism, 2-methylbutanoyl-CoA(4-) degradation Definition: The chemical reactions and pathways resulting in the breakdown of 2-methylbutanoyl-CoA(4-). Relationships: is a type of fatty-acyl-CoA catabolic process [GO:0036115]